amino sugar biosynthetic process [GO:0046349] (BP) Definition: The chemical reactions and pathways resulting in the formation of any amino sugar, sugars containing an amino group in place of a hydroxyl group. Sources: GOC:curators Also known as: amino sugar anabolism, amino sugar biosynthesis, amino sugar formation, amino sugar synthesis, aminosaccharide biosynthesis, aminosaccharide biosynthetic process Relationships: is a type of amino sugar metabolic process [GO:0006040]; is a type of carbohydrate derivative biosynthetic process [GO:1901137] Subtypes: UDP-N-acetylglucosamine biosynthetic process [GO:0006048], UDP-N-acetylgalactosamine biosynthetic process [GO:0019277], GO:0030391, mannosamine biosynthetic process [GO:0046347], GO:0046380, GO:1901073, UDP-4-deoxy-4-formamido-beta-L-arabinopyranose biosynthetic process [GO:2001315]